{
  "gene_name": "Villin-1",
  "term_label": "actin filament binding",
  "gene": "UniProtKB:P09327",
  "gene_symbol": "VIL1",
  "term_id": "GO:0051015"
}